{
  "gene": "UniProtKB:Q6PXP3",
  "gene_symbol": "SLC2A7",
  "term_label": "plasma membrane",
  "term_id": "GO:0005886",
  "gene_name": "Solute carrier family 2, facilitated glucose transporter member 7"
}